{
  "gene_name": "Myosin regulatory light polypeptide 9",
  "gene_symbol": "MYL9",
  "gene": "UniProtKB:P24844",
  "term_label": "myofibril assembly",
  "term_id": "GO:0030239"
}